{
  "gene": "UniProtKB:Q9Y6Y8",
  "gene_symbol": "SEC23IP",
  "term_id": "GO:0030134",
  "term_label": "COPII-coated ER to Golgi transport vesicle",
  "gene_name": "SEC23-interacting protein"
}